arsonoacetate metabolic process [GO:0018872] (biological process) Definition: The chemical reactions and pathways involving arsonoacetate, a synthetic, organic compound containing a single arsenic atom. Arsonoacetate and other arsenic containing compounds are used in agricultural applications as animal feed additives, cotton defoliants and post-emergence grass herbicides. Sources: UM-BBD_pathwayID:ara Also known as: arsonoacetate metabolism Relationships: is a type of GO:0006805; is a type of carboxylic acid metabolic process [GO:0019752] Subtypes: arsonoacetate catabolic process [GO:0019501]